L-histidine metabolic process [GO:0006547] (biological process) Definition: The chemical reactions and pathways involving L-histidine, 2-amino-3-(1H-imidazol-4-yl)propanoic acid. Sources: GOC:go_curators Also known as: histidine metabolic process, histidine metabolism Relationships: is a type of aromatic amino acid metabolic process [GO:0009072]; is a type of imidazole-containing compound metabolic process [GO:0052803]; is a type of L-amino acid metabolic process [GO:0170033]; is a type of proteinogenic amino acid metabolic process [GO:0170039] Subtypes: L-histidine biosynthetic process [GO:0000105], L-histidine catabolic process [GO:0006548]